voltage-gated potassium channel complex [GO:0008076] (cellular component) Relationships: is a type of potassium channel complex [GO:0034705]; is a type of plasma membrane protein complex [GO:0098797] Subtypes: GO:0071192, GO:0071193, Kv4.2-KChIP3 channel complex [GO:0071194], Kv4.2-KChIP4 channel complex [GO:0071195], GO:0071196, Kv4.2-Kv4.3 channel complex [GO:0071197], Kv4.1-DPP6 channel complex [GO:0071198], Kv4.1-DPP10 channel complex [GO:0071199], Kv4.2-DPP6 channel complex [GO:0071200], Kv4.3-DPP6 channel complex [GO:0071201], Kv4.3-DPP10 channel complex [GO:0071202], GO:0098855, inward rectifier potassium channel complex [GO:1902937] Sources: GOC:mah Also known as: voltage gated potassium channel complex, voltage-dependent potassium channel complex, voltage-sensitive potassium channel complex Definition: A protein complex that forms a transmembrane channel through which potassium ions may cross a cell membrane in response to changes in membrane potential.